seed dehydration [GO:1990068] (biological process) Definition: The seed development process whose outcome is the drying of a maturing seed. References: PMID:20138563 Relationships: is a type of multicellular organismal reproductive process [GO:0048609]; is part of seed maturation [GO:0010431]